nicotinamide riboside biosynthetic process [GO:0071590] (biological process) Definition: The chemical reactions and pathways resulting in the formation of nicotinamide riboside, the product of the formation of a glycosidic bond between ribose and nicotinamide. References: PMID:19846558 Sources: GOC:mah Also known as: N-ribosylnicotinamide biosynthetic process, nicotinamide riboside anabolism, nicotinamide riboside biosynthesis, nicotinamide riboside formation, nicotinamide riboside synthesis Relationships: is a type of nicotinamide riboside metabolic process [GO:0046495]; is a type of GO:0071589